alpha-amylase inhibitor activity [GO:0015066] (molecular function) Sources: GOC:mah Relationships: is a type of enzyme inhibitor activity [GO:0004857]; negatively regulates GO:0004556 Definition: Binds to and stops, prevents or reduces the activity of alpha-amylase.